{
  "gene": "UniProtKB:Q6P5X7",
  "term_id": "UNKNOWN:0002",
  "term_label": "Unknown biological process",
  "gene_symbol": "TMEM71",
  "gene_name": "Transmembrane protein 71"
}